{
  "gene_name": "Cyclin-dependent kinase-like 4",
  "gene_symbol": "CDKL4",
  "term_label": "nucleus",
  "term_id": "GO:0005634",
  "gene": "UniProtKB:Q5MAI5"
}